{
  "term_id": "UNKNOWN:0001",
  "gene": "UniProtKB:Q6ZU64",
  "gene_name": "Cilia- and flagella-associated protein 65",
  "term_label": "Unknown molecular function",
  "gene_symbol": "CFAP65"
}